{
  "term_label": "protein deubiquitination involved in ubiquitin-dependent protein catabolic process",
  "gene_symbol": "OTUD7B",
  "term_id": "GO:0071947",
  "gene": "UniProtKB:Q6GQQ9",
  "gene_name": "OTU domain-containing protein 7B"
}